{
  "gene_symbol": "MYL2",
  "term_id": "GO:0007507",
  "gene": "UniProtKB:P10916",
  "term_label": "heart development",
  "gene_name": "Myosin regulatory light chain 2, ventricular_cardiac muscle isoform"
}